dUMP metabolic process [GO:0046078] (biological process) Relationships: is a type of pyrimidine deoxyribonucleoside monophosphate metabolic process [GO:0009176]; is a type of pyrimidine deoxyribonucleotide metabolic process [GO:0009219] Sources: GOC:go_curators Definition: The chemical reactions and pathways involving dUMP, deoxyuridine (5'-)monophosphate (2'-deoxyuridine 5'-phosphate). Also known as: dUMP metabolism Subtypes: dUMP biosynthetic process [GO:0006226], dUMP catabolic process [GO:0046079]